{
  "gene": "UniProtKB:P22087",
  "gene_name": "rRNA 2'-O-methyltransferase fibrillarin",
  "gene_symbol": "FBL",
  "term_label": "rRNA methyltransferase activity",
  "term_id": "GO:0008649"
}